{
  "term_label": "somatic hypermutation of immunoglobulin genes",
  "gene_name": "Abasic site processing protein HMCES",
  "gene_symbol": "HMCES",
  "gene": "UniProtKB:Q96FZ2",
  "term_id": "GO:0016446"
}